{
  "gene_symbol": "SPATS2L",
  "term_id": "UNKNOWN:0001",
  "gene_name": "SPATS2-like protein",
  "term_label": "Unknown molecular function",
  "gene": "UniProtKB:Q9NUQ6"
}